{
  "term_label": "cell adhesion",
  "term_id": "GO:0007155",
  "gene_name": "Claudin-9",
  "gene": "UniProtKB:O95484",
  "gene_symbol": "CLDN9"
}